{
  "gene_symbol": "EXOSC9",
  "term_label": "exonucleolytic trimming to generate mature 3'-end of 5.8S rRNA from tricistronic rRNA transcript (SSU-rRNA, 5.8S rRNA, LSU-rRNA)",
  "term_id": "GO:0000467",
  "gene_name": "Exosome complex component RRP45",
  "gene": "UniProtKB:Q06265"
}